{
  "term_id": "GO:0007417",
  "gene_symbol": "SMO",
  "term_label": "central nervous system development",
  "gene_name": "Protein smoothened",
  "gene": "UniProtKB:Q99835"
}